regulation of cyclin-dependent protein serine/threonine kinase activity [GO:0000079] (BP) Definition: Any process that modulates the frequency, rate or extent of cyclin-dependent protein serine/threonine kinase activity. Subtypes: negative regulation of cyclin-dependent protein serine/threonine kinase activity [GO:0045736], positive regulation of cyclin-dependent protein serine/threonine kinase activity [GO:0045737] Relationships: is a type of regulation of protein serine/threonine kinase activity [GO:0071900]; regulates cyclin-dependent protein serine/threonine kinase activity [GO:0004693] Also known as: regulation of cyclin-dependent protein kinase activity, regulation of CDK activity Sources: GOC:go_curators, GOC:pr